{
  "term_id": "GO:0005886",
  "term_label": "plasma membrane",
  "gene": "UniProtKB:Q99788",
  "gene_symbol": "CMKLR1",
  "gene_name": "Chemerin-like receptor 1"
}